{
  "term_id": "GO:0000122",
  "gene": "UniProtKB:Q96HZ4",
  "gene_symbol": "HES6",
  "gene_name": "Transcription cofactor HES-6",
  "term_label": "negative regulation of transcription by RNA polymerase II"
}